{
  "term_id": "GO:0005886",
  "term_label": "plasma membrane",
  "gene_name": "Sorting nexin-4",
  "gene_symbol": "SNX4",
  "gene": "UniProtKB:O95219"
}